{
  "gene": "UniProtKB:O00155",
  "gene_symbol": "GPR25",
  "gene_name": "Probable G-protein coupled receptor 25",
  "term_id": "GO:0004930",
  "term_label": "G protein-coupled receptor activity"
}